{
  "gene": "UniProtKB:Q9NQV7",
  "gene_name": "Histone-lysine N-methyltransferase PRDM9",
  "term_id": "GO:0046975",
  "term_label": "histone H3K36 methyltransferase activity",
  "gene_symbol": "PRDM9"
}